{
  "gene": "UniProtKB:Q96DN2",
  "gene_name": "von Willebrand factor C and EGF domain-containing protein",
  "gene_symbol": "VWCE",
  "term_label": "Unknown molecular function",
  "term_id": "UNKNOWN:0001"
}